{
  "gene_name": "Zinc finger protein 117",
  "gene_symbol": "ZNF117",
  "gene": "UniProtKB:Q03924",
  "term_id": "GO:0000978",
  "term_label": "RNA polymerase II cis-regulatory region sequence-specific DNA binding"
}